{
  "gene_symbol": "CPD",
  "term_id": "GO:0004181",
  "term_label": "metallocarboxypeptidase activity",
  "gene": "UniProtKB:O75976",
  "gene_name": "Carboxypeptidase D"
}